{
  "term_id": "GO:0006357",
  "gene_name": "Doublesex- and mab-3-related transcription factor B1",
  "gene": "UniProtKB:Q96MA1",
  "term_label": "regulation of transcription by RNA polymerase II",
  "gene_symbol": "DMRTB1"
}